{
  "gene_symbol": "YTHDF1",
  "gene_name": "YTH domain-containing family protein 1",
  "term_id": "GO:1990247",
  "gene": "UniProtKB:Q9BYJ9",
  "term_label": "N6-methyladenosine-containing RNA reader activity"
}